{
  "term_label": "inflammatory response",
  "gene": "UniProtKB:P55774",
  "term_id": "GO:0006954",
  "gene_name": "C-C motif chemokine 18",
  "gene_symbol": "CCL18"
}